neurotransmitter receptor activity involved in regulation of presynaptic cytosolic calcium ion concentration [GO:0099582] (molecular function) Definition: Any neurotransmitter receptor activity that is involved in regulating the concentration of calcium in the presynaptic cytosol. Sources: GOC:dos Also known as: neurotransmitter receptor activity involved in regulation of presynaptic cytosolic calcium levels Relationships: is a type of neurotransmitter receptor activity [GO:0030594]; is part of regulation of presynaptic cytosolic calcium ion concentration [GO:0099509]; occurs in presynaptic membrane [GO:0042734]